{
  "gene_name": "Golgin subfamily A member 6A",
  "gene": "UniProtKB:Q9NYA3",
  "term_id": "GO:0000137",
  "term_label": "Golgi cis cisterna",
  "gene_symbol": "GOLGA6A"
}